{
  "term_label": "Unknown biological process",
  "gene_name": "Thyroxine-binding globulin",
  "term_id": "UNKNOWN:0002",
  "gene": "UniProtKB:P05543",
  "gene_symbol": "SERPINA7"
}